{
  "gene": "UniProtKB:Q13477",
  "gene_name": "Mucosal addressin cell adhesion molecule 1",
  "term_id": "GO:0034113",
  "term_label": "heterotypic cell-cell adhesion",
  "gene_symbol": "MADCAM1"
}